positive regulation of maintenance of meiotic sister chromatid cohesion, centromeric [GO:2000711] (biological process) Sources: GOC:mah Also known as: positive regulation of maintenance of centromeric meiotic sister chromatin cohesion, positive regulation of maintenance of meiotic sister chromatin cohesion at centromere, positive regulation of maintenance of sister chromatin cohesion at centromere at meiosis I Relationships: is a type of positive regulation of maintenance of meiotic sister chromatid cohesion [GO:0034096]; is a type of regulation of maintenance of meiotic sister chromatid cohesion, centromeric [GO:2000709]; positively regulates maintenance of meiotic sister chromatid cohesion, centromeric [GO:0035875] Definition: Any process that activates or increases the frequency, rate or extent of maintenance of meiotic sister chromatid cohesion in the centromeric region.